{
  "gene_name": "Cadherin-17",
  "term_label": "adherens junction organization",
  "gene_symbol": "CDH17",
  "term_id": "GO:0034332",
  "gene": "UniProtKB:Q12864"
}